{
  "term_id": "GO:0016477",
  "gene": "UniProtKB:Q93008",
  "gene_symbol": "USP9X",
  "gene_name": "Probable ubiquitin carboxyl-terminal hydrolase FAF-X",
  "term_label": "cell migration"
}